synaptic vesicle protein transport vesicle [GO:0097547] (cellular component) Note: This term should not be confused with GO:0008021 'synaptic vesicle'. STVs and synaptic vesicles differ both functionally and morphologically. Functionally, STVs are transport vesicles that deliver synaptic vesicle proteins to synapses, while synaptic vesicles are responsible for transmitter release at synapses. Morphologically, synaptic vesicles are very homogeneous, while STVs are very heterogeneous in size and shape. STVs might be a precursor for synaptic vesicles. Also known as: STV Relationships: is a type of cytoplasmic vesicle [GO:0031410] References: PMID:21569270 Sources: GOC:dr Definition: A cytoplasmic vesicle composed of both tubulovesicular and clear core vesicles that transport synaptic vesicle-associated proteins. Proteins carried by synaptic vesicle protein transport vesicles (STVs) include synaptophysin, synapsin Ia, synaptotagmin and synaptobrevin/vesicle-associated membrane protein 2 (VAMP2). STVs are packaged via the trans-Golgi network before being transported through the axon.